{
  "term_id": "UNKNOWN:0002",
  "gene_name": "Ciliary rootlet coiled-coil protein 2",
  "term_label": "Unknown biological process",
  "gene": "UniProtKB:H7BZ55",
  "gene_symbol": "CROCC2"
}